{
  "term_id": "UNKNOWN:0001",
  "gene_name": "Protein KTI12 homolog",
  "gene_symbol": "KTI12",
  "gene": "UniProtKB:Q96EK9",
  "term_label": "Unknown molecular function"
}